{
  "gene_symbol": "KCTD10",
  "gene": "UniProtKB:Q9H3F6",
  "gene_name": "BTB_POZ domain-containing adapter for CUL3-mediated RhoA degradation protein 3",
  "term_id": "GO:0031463",
  "term_label": "Cul3-RING ubiquitin ligase complex"
}